{
  "term_id": "UNKNOWN:0001",
  "term_label": "Unknown molecular function",
  "gene_symbol": "MTFR2",
  "gene": "UniProtKB:Q6P444",
  "gene_name": "Mitochondrial fission regulator 2"
}